{
  "gene_name": "Solute carrier family 35 member G6",
  "gene_symbol": "SLC35G6",
  "term_id": "UNKNOWN:0002",
  "gene": "UniProtKB:P0C7Q6",
  "term_label": "Unknown biological process"
}